{
  "gene_symbol": "ATP8A1",
  "term_id": "GO:0005886",
  "gene": "UniProtKB:Q9Y2Q0",
  "term_label": "plasma membrane",
  "gene_name": "Phospholipid-transporting ATPase IA"
}